positive regulation of calcium ion-dependent exocytosis of neurotransmitter [GO:1903235] (BP) Also known as: up regulation of calcium ion-dependent exocytosis of neurotransmitter, up-regulation of calcium ion-dependent exocytosis of neurotransmitter, upregulation of calcium ion-dependent exocytosis of neurotransmitter, activation of calcium ion-dependent exocytosis of neurotransmitter Definition: Any process that activates or increases the frequency, rate or extent of calcium ion-dependent exocytosis of neurotransmitter. References: PMID:16782817 Sources: GOC:TermGenie, GO_REF:0000058 Note: An example of this is Rab3gap1 in mouse (Q80UJ7) in PMID:16782817 (IMP) Relationships: is a type of GO:0045956; is a type of regulation of calcium ion-dependent exocytosis of neurotransmitter [GO:1903233]; is a type of GO:2000302; positively regulates GO:0048791